{
  "term_id": "GO:0005739",
  "gene": "UniProtKB:P52758",
  "gene_name": "2-iminobutanoate_2-iminopropanoate deaminase",
  "gene_symbol": "RIDA",
  "term_label": "mitochondrion"
}